{
  "term_id": "UNKNOWN:0003",
  "gene_symbol": "PYCARD-AS1",
  "gene": "UniProtKB:I3L0S3",
  "term_label": "Unknown cellular component",
  "gene_name": "Putative uncharacterized protein PYCARD-AS1"
}